{
  "gene_symbol": "CFAP20",
  "term_id": "GO:0060296",
  "gene_name": "Cilia- and flagella-associated protein 20",
  "term_label": "regulation of cilium beat frequency involved in ciliary motility",
  "gene": "UniProtKB:Q9Y6A4"
}